{
  "term_label": "Unknown biological process",
  "term_id": "UNKNOWN:0002",
  "gene_name": "Acyl-coenzyme A thioesterase 13",
  "gene": "UniProtKB:Q9NPJ3",
  "gene_symbol": "ACOT13"
}